fucosyltransferase activity [GO:0008417] (MF) Definition: Catalysis of the transfer of a fucosyl group to an acceptor molecule, typically another carbohydrate or a lipid. Sources: GOC:ai Subtypes: GO:0017060, alpha-(1,2)-fucosyltransferase activity [GO:0031127], alpha-(1->3)-fucosyltransferase activity [GO:0046920], alpha-(1->6)-fucosyltransferase activity [GO:0046921], peptide-O-fucosyltransferase activity [GO:0046922] Relationships: is a type of GO:0016758